{
  "term_id": "GO:0005543",
  "term_label": "phospholipid binding",
  "gene": "UniProtKB:O95208",
  "gene_symbol": "EPN2",
  "gene_name": "Epsin-2"
}